mitotic spindle pole body attachment site [GO:0180028] (cellular component) References: PMID:37783794 Definition: A region of the nuclear envelope to which a spindle pole body (SPB) attaches; protein complexes embedded in the nuclear envelope mediate direct or indirect linkages between the microtubule cytoskeleton and the nuclear envelope. Relationships: is a type of microtubule organizing center attachment site [GO:0034992]